{
  "gene": "UniProtKB:P51787",
  "gene_symbol": "KCNQ1",
  "term_label": "membrane repolarization during ventricular cardiac muscle cell action potential",
  "term_id": "GO:0098915",
  "gene_name": "Potassium voltage-gated channel subfamily KQT member 1"
}